meiosis I nuclear membrane disassembly [GO:0051079] (biological process) Relationships: is a type of meiotic nuclear membrane disassembly [GO:0051078]; is part of GO:0007127 Definition: The controlled breakdown of the nuclear membranes during the first division of meiosis. Also known as: meiosis I nuclear envelope breakdown, meiosis I nuclear envelope catabolism, meiosis I nuclear envelope degradation, meiosis I nuclear envelope disassembly Sources: GOC:bf